{
  "term_label": "mRNA cis splicing, via spliceosome",
  "term_id": "GO:0045292",
  "gene_name": "Methylosome subunit pICln",
  "gene_symbol": "CLNS1A",
  "gene": "UniProtKB:P54105"
}